{
  "gene_name": "Putative uncharacterized protein FLJ26174",
  "term_label": "Unknown cellular component",
  "gene": "UniProtKB:Q6ZPA2",
  "term_id": "UNKNOWN:0003",
  "gene_symbol": "Q6ZPA2"
}